{
  "gene_name": "Cytochrome P450 4F2",
  "gene": "UniProtKB:P78329",
  "term_id": "UNKNOWN:0001",
  "gene_symbol": "CYP4F2",
  "term_label": "Unknown molecular function"
}